response to N-acetyl-D-glucosamine [GO:0097315] (biological process) Definition: Any process that results in a change in state or activity of a cell or an organism (in terms of movement, secretion, enzyme production, gene expression, etc.) as a result of an N-acetyl-D-glucosamine stimulus. Subtypes: cellular response to N-acetyl-D-glucosamine [GO:0097316] References: PMID:21700702 Sources: GOC:di Relationships: is a type of response to oxygen-containing compound [GO:1901700]